chloramphenicol transmembrane transporter activity [GO:0042896] (molecular function) Definition: Enables the transfer of chloramphenicol, a broad-spectrum antibiotic that inhibits bacterial protein synthesis, from one side of a membrane to the other. Sources: GOC:jl Also known as: chloramphenicol transporter activity Relationships: is a type of polyol transmembrane transporter activity [GO:0015166]; is a type of amide transmembrane transporter activity [GO:0042887]; is part of chloramphenicol transmembrane transport [GO:0042892]